{
  "term_id": "GO:0005783",
  "gene_symbol": "ATP2C1",
  "gene": "UniProtKB:P98194",
  "term_label": "endoplasmic reticulum",
  "gene_name": "Calcium-transporting ATPase type 2C member 1"
}